{
  "term_label": "spindle pole",
  "gene": "UniProtKB:Q96EA4",
  "gene_symbol": "SPDL1",
  "term_id": "GO:0000922",
  "gene_name": "Protein Spindly"
}